distinct antral spaces stage [GO:0048164] (BP) Also known as: mammalian oogenesis stage 7 Sources: GOC:jid, GOC:mtg_sensu, ISBN:0198542771 Relationships: is a type of mammalian oogenesis stage [GO:0022605] Definition: The stage in oogenesis when the antral spaces become distinct and the first polar body forms.